{
  "term_label": "regulation of transcription by RNA polymerase II",
  "gene_symbol": "NFYB",
  "gene": "UniProtKB:P25208",
  "term_id": "GO:0006357",
  "gene_name": "Nuclear transcription factor Y subunit beta"
}